{
  "gene_symbol": "XRCC1",
  "term_id": "GO:0006284",
  "gene_name": "DNA repair protein XRCC1",
  "gene": "UniProtKB:P18887",
  "term_label": "base-excision repair"
}